{
  "gene_name": "Group IIF secretory phospholipase A2",
  "gene": "UniProtKB:Q9BZM2",
  "gene_symbol": "PLA2G2F",
  "term_id": "GO:0046471",
  "term_label": "phosphatidylglycerol metabolic process"
}